{
  "term_id": "UNKNOWN:0003",
  "gene_name": "WD repeat and SOCS box-containing protein 1",
  "gene": "UniProtKB:Q9Y6I7",
  "term_label": "Unknown cellular component",
  "gene_symbol": "WSB1"
}